{
  "gene_name": "Tryptase delta",
  "gene": "UniProtKB:Q9BZJ3",
  "term_label": "serine-type endopeptidase activity",
  "term_id": "GO:0004252",
  "gene_symbol": "TPSD1"
}